{
  "gene_name": "GDP-fucose protein O-fucosyltransferase 1",
  "term_label": "protein O-linked glycosylation via fucose",
  "gene_symbol": "POFUT1",
  "term_id": "GO:0036066",
  "gene": "UniProtKB:Q9H488"
}